{
  "gene_symbol": "SOX10",
  "gene_name": "Transcription factor SOX-10",
  "term_label": "neural crest cell migration",
  "gene": "UniProtKB:P56693",
  "term_id": "GO:0001755"
}